{
  "gene": "UniProtKB:Q9Y603",
  "gene_symbol": "ETV7",
  "gene_name": "Transcription factor ETV7",
  "term_label": "regulation of transcription by RNA polymerase II",
  "term_id": "GO:0006357"
}